{
  "term_label": "Unknown cellular component",
  "gene_symbol": "MEA1",
  "gene": "UniProtKB:Q16626",
  "gene_name": "Male-enhanced antigen 1",
  "term_id": "UNKNOWN:0003"
}